{
  "term_id": "GO:0002098",
  "gene_symbol": "ALKBH8",
  "gene_name": "Alkylated DNA repair protein alkB homolog 8",
  "gene": "UniProtKB:Q96BT7",
  "term_label": "tRNA wobble uridine modification"
}